negative regulation of secretory granule organization [GO:1904410] (biological process) Also known as: down regulation of secretory granule organisation, down regulation of secretory granule organization, down-regulation of secretory granule organisation, down-regulation of secretory granule organization, downregulation of secretory granule organisation, downregulation of secretory granule organization, negative regulation of secretory granule organisation, inhibition of secretory granule organisation, inhibition of secretory granule organization, down regulation of secretory granule organization and biogenesis, down-regulation of secretory granule organization and biogenesis, downregulation of secretory granule organization and biogenesis, inhibition of secretory granule organization and biogenesis, negative regulation of secretory granule organization and biogenesis References: PMID:15039777 Sources: GOC:TermGenie, GO_REF:0000058 Definition: Any process that stops, prevents or reduces the frequency, rate or extent of secretory granule organization. Relationships: is a type of negative regulation of organelle organization [GO:0010639]; is a type of regulation of secretory granule organization [GO:1904409]; negatively regulates GO:0033363